tRNA wobble base 5-methoxycarbonylmethyl-2-thiouridinylation [GO:0002926] (biological process) Definition: The process whereby a wobble base uridine residue in a tRNA is modified to 5-methoxycarbonylmethyl-2-thiouridine. References: PMID:22768388 Sources: GOC:hjd Relationships: is a type of tRNA wobble uridine modification [GO:0002098] Also known as: mcm5 modification, mcm5s2U34 biosynthesis, tRNA wobble base 5-methoxycarbonylmethyl-2-thiouridine biosynthesis